{
  "gene_name": "Homeobox protein GBX-1",
  "gene_symbol": "GBX1",
  "gene": "UniProtKB:Q14549",
  "term_id": "GO:0000981",
  "term_label": "DNA-binding transcription factor activity, RNA polymerase II-specific"
}